{
  "term_id": "GO:0000978",
  "gene_name": "Forkhead box protein Q1",
  "gene": "UniProtKB:Q9C009",
  "term_label": "RNA polymerase II cis-regulatory region sequence-specific DNA binding",
  "gene_symbol": "FOXQ1"
}